{
  "term_label": "Unknown molecular function",
  "term_id": "UNKNOWN:0001",
  "gene_symbol": "POM121L1P",
  "gene_name": "Putative POM121-like protein 1",
  "gene": "UniProtKB:Q3SYA9"
}